{
  "term_id": "GO:0005739",
  "gene": "UniProtKB:Q96I99",
  "gene_name": "Succinate--CoA ligase [GDP-forming] subunit beta, mitochondrial",
  "gene_symbol": "SUCLG2",
  "term_label": "mitochondrion"
}